{
  "term_label": "spliceosomal complex disassembly",
  "gene": "UniProtKB:Q9NVM6",
  "term_id": "GO:0000390",
  "gene_symbol": "DNAJC17",
  "gene_name": "DnaJ homolog subfamily C member 17"
}